{
  "gene_name": "1-phosphatidylinositol 4,5-bisphosphate phosphodiesterase zeta-1",
  "gene": "UniProtKB:Q86YW0",
  "gene_symbol": "PLCZ1",
  "term_id": "GO:0005634",
  "term_label": "nucleus"
}